negative regulation of type IV hypersensitivity [GO:0001808] (biological process) Sources: GOC:add, ISBN:0781735149 Relationships: is a type of regulation of type IV hypersensitivity [GO:0001807]; is a type of negative regulation of T cell mediated immunity [GO:0002710]; is a type of negative regulation of hypersensitivity [GO:0002884]; negatively regulates type IV hypersensitivity [GO:0001806] Also known as: down regulation of type IV hypersensitivity, down-regulation of type IV hypersensitivity, downregulation of type IV hypersensitivity, inhibition of type IV hypersensitivity Definition: Any process that stops, prevents, or reduces the rate of type IV hypersensitivity, a type of inflammatory response.